{
  "term_id": "GO:0042805",
  "term_label": "actinin binding",
  "gene_name": "Cysteine and glycine-rich protein 2",
  "gene_symbol": "CSRP2",
  "gene": "UniProtKB:Q16527"
}